polyol catabolic process [GO:0046174] (BP) Subtypes: inositol catabolic process [GO:0019310], alditol catabolic process [GO:0019405], diol catabolic process [GO:0034313], inositol phosphate catabolic process [GO:0071545], tobramycin catabolic process [GO:1901120], GO:1901129, kanamycin catabolic process [GO:1901132], vistamycin catabolic process [GO:1901151], paromomycin catabolic process [GO:1901154], neomycin catabolic process [GO:1901157], GO:1901743, GO:1901757, GO:1901802 Definition: The chemical reactions and pathways resulting in the breakdown of a polyol, any alcohol containing three or more hydroxyl groups attached to saturated carbon atoms. Relationships: is a type of polyol metabolic process [GO:0019751]; is a type of alcohol catabolic process [GO:0046164] Also known as: polyhydric alcohol catabolic process, polyol breakdown, polyol catabolism, polyol degradation Sources: GOC:curators